host intracellular organelle [GO:0033647] (cellular component) Relationships: is a type of host intracellular part [GO:0033646] Subtypes: host intracellular membrane-bounded organelle [GO:0033648], host thylakoid [GO:0044159], GO:0044163, host chromosome [GO:0044383] Sources: GOC:pamgo_curators Definition: Organized structure of distinctive morphology and function, occurring within the host cell. Includes the nucleus, mitochondria, plastids, vacuoles, vesicles, ribosomes and the cytoskeleton. Excludes the plasma membrane. The host is defined as the larger of the organisms involved in a symbiotic interaction.